tripeptide aminopeptidase activity [GO:0045148] (molecular function) Also known as: aminotripeptidase activity, peptidase T, alanine-phenylalanine-proline arylamidase activity, aminoexotripeptidase activity, imidoendopeptidase activity, lymphopeptidase activity, peptidase B Relationships: is a type of aminopeptidase activity [GO:0004177]; is a type of GO:0034701 Sources: EC:3.4.11.4 Definition: Catalysis of the hydrolysis of a single N-terminal amino acid residue from a tripeptide.